{
  "gene_symbol": "CSRNP1",
  "gene": "UniProtKB:Q96S65",
  "term_label": "nucleus",
  "term_id": "GO:0005634",
  "gene_name": "Cysteine_serine-rich nuclear protein 1"
}